{
  "gene_symbol": "LYN",
  "term_label": "signaling receptor binding",
  "term_id": "GO:0005102",
  "gene": "UniProtKB:P07948",
  "gene_name": "Tyrosine-protein kinase Lyn"
}